{
  "gene": "UniProtKB:Q14457",
  "gene_symbol": "BECN1",
  "gene_name": "Beclin-1",
  "term_label": "late endosome to vacuole transport",
  "term_id": "GO:0045324"
}